{
  "gene_name": "Phosphatidylinositol 3,4,5-trisphosphate 3-phosphatase and dual-specificity protein phosphatase PTEN",
  "term_id": "GO:0051896",
  "gene": "UniProtKB:P60484",
  "term_label": "regulation of phosphatidylinositol 3-kinase/protein kinase B signal transduction",
  "gene_symbol": "PTEN"
}